{
  "term_id": "GO:0031267",
  "gene_symbol": "RINL",
  "term_label": "small GTPase binding",
  "gene": "UniProtKB:Q6ZS11",
  "gene_name": "Ras and Rab interactor-like protein"
}